{
  "gene_name": "Endoribonuclease LACTB2",
  "gene": "UniProtKB:Q53H82",
  "gene_symbol": "LACTB2",
  "term_id": "GO:0005759",
  "term_label": "mitochondrial matrix"
}